{
  "gene": "UniProtKB:Q9UHF1",
  "term_label": "extracellular region",
  "gene_symbol": "EGFL7",
  "term_id": "GO:0005576",
  "gene_name": "Epidermal growth factor-like protein 7"
}